{
  "gene": "UniProtKB:Q9BTL4",
  "gene_symbol": "IER2",
  "gene_name": "Immediate early response gene 2 protein",
  "term_label": "Unknown molecular function",
  "term_id": "UNKNOWN:0001"
}